{
  "gene": "UniProtKB:Q9NQ36",
  "gene_name": "Signal peptide, CUB and EGF-like domain-containing protein 2",
  "gene_symbol": "SCUBE2",
  "term_id": "GO:0009986",
  "term_label": "cell surface"
}